{
  "gene": "UniProtKB:P51575",
  "term_id": "GO:0004931",
  "gene_name": "P2X purinoceptor 1",
  "term_label": "extracellularly ATP-gated monoatomic cation channel activity",
  "gene_symbol": "P2RX1"
}